phosphoribokinase activity [GO:0050195] (molecular function) Definition: Catalysis of the reaction: D-ribose 5-phosphate + ATP = D-ribose 1,5-diphosphate + ADP + 2 H+. Relationships: is a type of kinase activity [GO:0016301]; is a type of phosphotransferase activity, alcohol group as acceptor [GO:0016773] Also known as: ATP:D-ribose-5-phosphate 1-phosphotransferase activity, phosphoribokinase (phosphorylating) Sources: EC:2.7.1.18, RHEA:21216